endospore formation [GO:0034301] (biological process) Relationships: is a type of asexual sporulation resulting in formation of a cellular spore [GO:0043936] Definition: The process in which a cell gives rise to an endospore, a dormant, highly resistant spore with a thick wall that forms within the mother cell. Endospores are produced by some low G+C Gram-positive bacteria in response to harsh conditions. Sources: GOC:ds, GOC:mah, ISBN:0470090278